{
  "term_label": "Unknown cellular component",
  "term_id": "UNKNOWN:0003",
  "gene_symbol": "GOLGA6L4",
  "gene": "UniProtKB:A6NEF3",
  "gene_name": "Golgin subfamily A member 6-like protein 4"
}